{
  "gene": "UniProtKB:Q8N5U1",
  "gene_symbol": "MS4A15",
  "gene_name": "Membrane-spanning 4-domains subfamily A member 15",
  "term_id": "GO:0005886",
  "term_label": "plasma membrane"
}